{
  "gene_symbol": "SNX17",
  "gene": "UniProtKB:Q15036",
  "term_id": "GO:0006886",
  "gene_name": "Sorting nexin-17",
  "term_label": "intracellular protein transport"
}